{
  "gene": "UniProtKB:P00973",
  "term_id": "GO:0045071",
  "term_label": "negative regulation of viral genome replication",
  "gene_symbol": "OAS1",
  "gene_name": "2'-5'-oligoadenylate synthase 1"
}